regulation of receptor signaling pathway via STAT [GO:1904892] (biological process) Also known as: regulation of STAT signalling pathway, regulation of kinase activated-STAT cascade, regulation of kinase-STAT cascade Definition: Any process that modulates the frequency, rate or extent of receptor signaling via STAT. References: PMID:24587195 Sources: GOC:TermGenie, GOC:rjd, GO_REF:0000058 Relationships: is a type of GO:0009966; regulates cell surface receptor signaling pathway via STAT [GO:0097696] Subtypes: regulation of receptor signaling pathway via JAK-STAT [GO:0046425], negative regulation of receptor signaling pathway via STAT [GO:1904893], GO:1904894